{
  "gene": "UniProtKB:P02746",
  "term_id": "UNKNOWN:0001",
  "term_label": "Unknown molecular function",
  "gene_name": "Complement C1q subcomponent subunit B",
  "gene_symbol": "C1QB"
}